{
  "gene_name": "Mucin-3B",
  "gene_symbol": "MUC3B",
  "gene": "UniProtKB:Q9H195",
  "term_label": "Unknown biological process",
  "term_id": "UNKNOWN:0002"
}